{
  "gene_symbol": "DDB1",
  "term_label": "proteasome-mediated ubiquitin-dependent protein catabolic process",
  "gene": "UniProtKB:Q16531",
  "term_id": "GO:0043161",
  "gene_name": "DNA damage-binding protein 1"
}